negative regulation of spore germination [GO:1904360] (biological process) Definition: Any process that stops, prevents or reduces the frequency, rate or extent of spore germination. References: PMID:14718564, PMID:8798577 Sources: GOC:TermGenie, GO_REF:0000058 Also known as: down regulation of spore germination, down-regulation of spore germination, downregulation of spore germination, inhibition of spore germination, negative regulation of spore germination on or near host Relationships: is a type of negative regulation of cellular process [GO:0048523]; is a type of negative regulation of developmental process [GO:0051093]; is_a regulation of spore germination [GO:1904359]; negatively regulates spore germination [GO:0009847] Subtypes: negative regulation of encysted zoospore germination [GO:0075229]